oxidoreductase activity, acting on X-H and Y-H to form an X-Y bond, with a disulfide as acceptor [GO:0050485] (molecular function) Also known as: oxidoreductase activity, acting on X-H and Y-H to form an X-Y bond, with a disulphide as acceptor Sources: EC:1.21.4.- Subtypes: GO:0030699, sarcosine reductase activity [GO:0033794], betaine reductase activity [GO:0033795], GO:0050002 Relationships: is a type of oxidoreductase activity, acting on X-H and Y-H to form an X-Y bond [GO:0046992] Definition: Catalysis of an oxidation-reduction (redox) reaction in which X-H and Y-H form X-Y and the acceptor is disulfide.